carboxynorspermidine dehydrogenase activity [GO:0102143] (molecular function) Sources: EC:1.5.1.43 Definition: Catalysis of the reaction: carboxynorspermidine + H2O + NADP+ = H+ + L-aspartate 4-semialdehyde + NADPH + propane-1,3-diamine. Also converts carboxyspermidine to putrescine. Relationships: is a type of oxidoreductase activity, acting on the CH-NH group of donors, NAD or NADP as acceptor [GO:0016646] Also known as: carboxynorspermidine dehydrogenase I activity, carboxynorspermidine dehydrogenase II activity